trochlear nerve development [GO:0021558] (biological process) Definition: The process whose specific outcome is the progression of the trochlear nerve over time, from its formation to the mature structure. The trochlear nerve is a motor nerve and is the only cranial nerve to exit the brain dorsally. The trochlear nerve innervates the superior oblique muscle. Sources: GOC:cls, GOC:dgh, GOC:dph, GOC:jid, GO_REF:0000021 Also known as: cranial nerve 4 development, cranial nerve IV development, CN IV development Relationships: is a type of cranial nerve development [GO:0021545]